positive regulation of central B cell tolerance induction [GO:0002897] (biological process) Definition: Any process that activates or increases the frequency, rate, or extent of central B cell tolerance induction. Relationships: is a type of positive regulation of central tolerance induction [GO:0002648]; is a type of GO:0002663; is a type of GO:0002895; positively regulates central B cell tolerance induction [GO:0002510] Also known as: up regulation of central B cell tolerance induction, up-regulation of central B cell tolerance induction, upregulation of central B cell tolerance induction, activation of central B cell tolerance induction, stimulation of central B cell tolerance induction Sources: GOC:add Subtypes: GO:0002900, positive regulation of central B cell anergy [GO:0002916]